iron ion export across plasma membrane [GO:1903988] (biological process) Also known as: ferrous iron export, ferrous iron export across plasma membrane, iron cation export, iron(2+) export Definition: The directed movement of iron ions from inside of a cell, across the plasma membrane and into the extracellular region. Relationships: is a type of iron ion transmembrane transport [GO:0034755]; is a type of export across plasma membrane [GO:0140115] Note: An example of this is mouse ferroportin (symbol Slc40a1, UniProtKB identifier: Q9JHI9). Regulation: regulated by regulation of iron export across plasma membrane [GO:1904038]; negatively regulated by negative regulation of iron export across plasma membrane [GO:1904039]; positively regulated by positive regulation of iron export across plasma membrane [GO:1904040] References: PMID:15514116 Sources: GOC:BHF, GOC:TermGenie, GOC:kom, GOC:rl, GO_REF:0000074